{
  "term_label": "Unknown biological process",
  "gene_name": "Nicotinamide N-methyltransferase",
  "term_id": "UNKNOWN:0002",
  "gene_symbol": "NNMT",
  "gene": "UniProtKB:P40261"
}